{
  "gene_name": "Coronin-7",
  "gene_symbol": "CORO7",
  "term_id": "GO:0035332",
  "gene": "UniProtKB:P57737",
  "term_label": "positive regulation of hippo signaling"
}